citric acid secretion [GO:0046720] (biological process) Relationships: is_a citrate transport [GO:0015746]; is a type of GO:0046717 Sources: GOC:ai Definition: The controlled release of citric acid, 2-hydroxy-1,2,3-propanetricarboxylic acid, by a cell or a tissue. Also known as: citrate secretion